PSII associated light-harvesting complex II [GO:0009517] (cellular component) Relationships: is a type of thylakoid light-harvesting complex [GO:0009503] Definition: Protein-pigment complex associated with photosystem II. Also known as: LHCII Sources: GOC:lr, ISBN:0582227089